leukocyte chemotaxis involved in immune response [GO:0002233] (biological process) Relationships: is a type of leukocyte migration involved in immune response [GO:0002522]; is a type of leukocyte chemotaxis [GO:0030595] Definition: The movement of an immune cell in response to an external stimulus a part of an immune response. Also known as: immune cell chemotaxis during immune response, leucocyte chemotaxis during immune response Sources: GOC:add, ISBN:0781735149